hopanoid biosynthetic process [GO:0019746] (biological process) Definition: The chemical reactions and pathways resulting in the formation of hopanoids, pentacyclic sterol-like compounds based on the hopane nucleus. Relationships: is a type of triterpenoid biosynthetic process [GO:0016104] Also known as: hopanoid anabolism, hopanoid biosynthesis, hopanoid formation, hopanoid synthesis Sources: ISBN:0198547684